{
  "term_id": "GO:0004523",
  "gene_symbol": "FEN1",
  "gene": "UniProtKB:P39748",
  "gene_name": "Flap endonuclease 1",
  "term_label": "RNA-DNA hybrid ribonuclease activity"
}